{
  "term_id": "GO:0005783",
  "gene": "UniProtKB:Q8NFQ8",
  "gene_symbol": "TOR1AIP2",
  "gene_name": "Torsin-1A-interacting protein 2",
  "term_label": "endoplasmic reticulum"
}